{
  "term_label": "recycling endosome membrane",
  "gene_symbol": "EHD4",
  "term_id": "GO:0055038",
  "gene_name": "EH domain-containing protein 4",
  "gene": "UniProtKB:Q9H223"
}